{
  "term_id": "UNKNOWN:0003",
  "gene": "UniProtKB:Q6P2I3",
  "gene_name": "Fumarylacetoacetate hydrolase domain-containing protein 2B",
  "term_label": "Unknown cellular component",
  "gene_symbol": "FAHD2B"
}